{
  "gene_name": "Glycine dehydrogenase (decarboxylating), mitochondrial",
  "gene_symbol": "GLDC",
  "gene": "UniProtKB:P23378",
  "term_id": "GO:0005739",
  "term_label": "mitochondrion"
}